{
  "term_label": "RNA polymerase II transcription regulatory region sequence-specific DNA binding",
  "term_id": "GO:0000977",
  "gene_symbol": "PTF1A",
  "gene_name": "Pancreas transcription factor 1 subunit alpha",
  "gene": "UniProtKB:Q7RTS3"
}